pyridoxal 5'-phosphate salvage [GO:0009443] (biological process) Sources: GOC:jl Subtypes: pyridoxal phosphate biosynthetic process from pyridoxamine [GO:0010144] Definition: Any process that generates pyridoxal 5'-phosphate, the active form of vitamin B6, from derivatives of it without de novo synthesis. Relationships: is a type of pyridoxal phosphate biosynthetic process [GO:0042823]; is a type of GO:0043094 Also known as: pyridoxal 5' phosphate salvage